{
  "gene": "UniProtKB:Q9Y3A4",
  "gene_symbol": "RRP7A",
  "term_id": "GO:0006364",
  "term_label": "rRNA processing",
  "gene_name": "Ribosomal RNA-processing protein 7 homolog A"
}